{
  "gene_symbol": "IPCEF1",
  "term_id": "UNKNOWN:0003",
  "gene": "UniProtKB:Q8WWN9",
  "term_label": "Unknown cellular component",
  "gene_name": "Interactor protein for cytohesin exchange factors 1"
}